{
  "gene": "UniProtKB:Q569H4",
  "gene_name": "Protein Largen",
  "term_label": "Unknown cellular component",
  "term_id": "UNKNOWN:0003",
  "gene_symbol": "PRR16"
}